neuromast hair cell differentiation [GO:0048886] (biological process) Sources: CL:0000856, ISBN:0125296509 Relationships: is a type of hair cell differentiation [GO:0035315]; is_a mechanoreceptor differentiation [GO:0042490]; is part of neuromast development [GO:0048884] Definition: The process in which a relatively unspecialized cell acquires specialized features of a neuromast hair cell. Hair cells are the sensory receptors of the neuromast and are located in a portion of the neuromast called the sensory strip. Each hair cell of the neuromast is morphologically polarized as a result of the relative position of the single kinocilium and the clusters of stereocilia on its apical surface. There are approximately seven hair cells within each neuromast, with each hair cell innervated by afferent and efferent neurons. Subtypes: anterior lateral line neuromast hair cell differentiation [GO:0048903], posterior lateral line neuromast hair cell differentiation [GO:0048923], neuromast hair cell differentiation involved in neuromast regeneration [GO:0070658]